{
  "term_label": "positive regulation of triglyceride storage",
  "term_id": "GO:0010890",
  "gene": "UniProtKB:Q99541",
  "gene_name": "Perilipin-2",
  "gene_symbol": "PLIN2"
}